{
  "gene": "UniProtKB:Q99619",
  "term_label": "cytosol",
  "term_id": "GO:0005829",
  "gene_symbol": "SPSB2",
  "gene_name": "SPRY domain-containing SOCS box protein 2"
}